{
  "gene_name": "Interferon-induced protein with tetratricopeptide repeats 2",
  "gene_symbol": "IFIT2",
  "gene": "UniProtKB:P09913",
  "term_id": "GO:0140374",
  "term_label": "antiviral innate immune response"
}